{
  "term_label": "Unknown cellular component",
  "gene_name": "Fertilization-influencing membrane protein",
  "gene": "UniProtKB:Q96LL3",
  "gene_symbol": "FIMP",
  "term_id": "UNKNOWN:0003"
}